cortisol binding [GO:1903794] (molecular function) References: PMID:18483153 Sources: GOC:TermGenie, GOC:mr, GO_REF:0000067 Relationships: is a type of alcohol binding [GO:0043178]; is a type of steroid hormone binding [GO:1990239] Definition: Binding to cortisol.